{
  "term_label": "plasma membrane",
  "term_id": "GO:0005886",
  "gene_name": "Cyclin-Y",
  "gene_symbol": "CCNY",
  "gene": "UniProtKB:Q8ND76"
}